3-beta-hydroxy-5-beta-steroid dehydrogenase (NADP+) activity [GO:0033703] (molecular function) Relationships: is a type of steroid dehydrogenase activity, acting on the CH-OH group of donors, NAD or NADP as acceptor [GO:0033764] Also known as: 3beta-hydroxy-5beta-steroid:NADP+ 3-oxidoreductase activity, 3beta-hydroxysteroid 5beta-oxidoreductase activity, 3beta-hydroxysteroid 5beta-progesterone oxidoreductase activity Definition: Catalysis of the reaction: 3-beta-hydroxy-5-beta-pregnane-20-one + NADP+ = 5-beta-pregnan-3,20-dione + H+ + NADPH. Sources: RHEA:22944